positive regulation of membrane potential [GO:0045838] (biological process) Definition: Any process that activates or increases the frequency, rate or extent of establishment or extent of a membrane potential, the electric potential existing across any membrane arising from charges in the membrane itself and from the charges present in the media on either side of the membrane. Also known as: elevation of membrane potential, up regulation of membrane potential, up-regulation of membrane potential, upregulation of membrane potential, activation of membrane potential, stimulation of membrane potential Subtypes: positive regulation of mitochondrial membrane potential [GO:0010918] Relationships: is a type of GO:0042391 Sources: GOC:go_curators